{
  "term_label": "chemical synaptic transmission",
  "gene": "UniProtKB:P30939",
  "term_id": "GO:0007268",
  "gene_name": "5-hydroxytryptamine receptor 1F",
  "gene_symbol": "HTR1F"
}